{
  "term_id": "UNKNOWN:0003",
  "term_label": "Unknown cellular component",
  "gene_symbol": "CT47C1",
  "gene": "UniProtKB:A0A0U1RQG5",
  "gene_name": "Cancer_testis antigen family 47 member C1"
}